{
  "gene_symbol": "NPIPB3",
  "term_label": "Unknown molecular function",
  "gene_name": "Nuclear pore complex-interacting protein family member B3",
  "gene": "UniProtKB:Q92617",
  "term_id": "UNKNOWN:0001"
}